{
  "term_label": "regulation of transcription by RNA polymerase II",
  "gene": "UniProtKB:Q9BQW3",
  "gene_name": "Transcription factor COE4",
  "gene_symbol": "EBF4",
  "term_id": "GO:0006357"
}